{
  "gene_symbol": "SPATA33",
  "gene_name": "Spermatogenesis-associated protein 33",
  "term_label": "Unknown molecular function",
  "term_id": "UNKNOWN:0001",
  "gene": "UniProtKB:Q96N06"
}